{
  "term_label": "intrinsic apoptotic signaling pathway in response to DNA damage by p53 class mediator",
  "gene": "UniProtKB:P04637",
  "gene_name": "Cellular tumor antigen p53",
  "gene_symbol": "TP53",
  "term_id": "GO:0042771"
}